{
  "gene_symbol": "ACADM",
  "term_label": "medium-chain fatty acyl-CoA dehydrogenase activity",
  "gene_name": "Medium-chain specific acyl-CoA dehydrogenase, mitochondrial",
  "gene": "UniProtKB:P11310",
  "term_id": "GO:0070991"
}